{
  "gene_symbol": "TGM5",
  "gene_name": "Protein-glutamine gamma-glutamyltransferase 5",
  "term_id": "GO:0018149",
  "gene": "UniProtKB:O43548",
  "term_label": "peptide cross-linking"
}